{
  "gene": "UniProtKB:Q13642",
  "term_label": "transmembrane transporter binding",
  "gene_symbol": "FHL1",
  "term_id": "GO:0044325",
  "gene_name": "Four and a half LIM domains protein 1"
}